{
  "gene_name": "Coatomer subunit gamma-1",
  "gene": "UniProtKB:Q9Y678",
  "gene_symbol": "COPG1",
  "term_label": "endoplasmic reticulum-Golgi intermediate compartment",
  "term_id": "GO:0005793"
}